{
  "gene_name": "Putative transcription factor Ovo-like 1",
  "term_label": "regulation of transcription by RNA polymerase II",
  "term_id": "GO:0006357",
  "gene_symbol": "OVOL1",
  "gene": "UniProtKB:O14753"
}